{
  "term_label": "synapse maturation",
  "term_id": "GO:0060074",
  "gene_name": "Seizure 6-like protein 2",
  "gene": "UniProtKB:Q6UXD5",
  "gene_symbol": "SEZ6L2"
}